positive regulation of presynaptic active zone assembly [GO:1905520] (biological process) Definition: Any process that activates or increases the frequency, rate or extent of presynaptic active zone assembly. References: PMID:15797875 Sources: GOC:BHF, GOC:TermGenie, GOC:rl, GO_REF:0000058 Also known as: positive regulation of pre-synaptic active zone assembly, positive regulation of pre-synaptic active zone formation, positive regulation of presynaptic active zone formation, up regulation of pre-synaptic active zone assembly, up regulation of pre-synaptic active zone formation, up regulation of presynaptic active zone assembly, up regulation of presynaptic active zone formation, up-regulation of pre-synaptic active zone assembly, up-regulation of pre-synaptic active zone formation, up-regulation of presynaptic active zone assembly, up-regulation of presynaptic active zone formation, upregulation of pre-synaptic active zone assembly, upregulation of pre-synaptic active zone formation, upregulation of presynaptic active zone assembly, upregulation of presynaptic active zone formation, activation of pre-synaptic active zone assembly, activation of pre-synaptic active zone component assembly, activation of pre-synaptic active zone component formation, activation of pre-synaptic active zone formation, activation of presynaptic active zone assembly, activation of presynaptic active zone formation, positive regulation of pre-synaptic active zone component assembly, positive regulation of pre-synaptic active zone component formation, up regulation of pre-synaptic active zone component assembly, up regulation of pre-synaptic active zone component formation, up-regulation of pre-synaptic active zone component assembly, up-regulation of pre-synaptic active zone component formation, upregulation of pre-synaptic active zone component assembly, upregulation of pre-synaptic active zone component formation Relationships: is a type of regulation of presynaptic active zone assembly [GO:1905518]; is a type of positive regulation of presynapse assembly [GO:1905608]; positively regulates presynaptic active zone assembly [GO:1904071]